{
  "gene": "UniProtKB:Q13085",
  "gene_symbol": "ACACA",
  "gene_name": "Acetyl-CoA carboxylase 1",
  "term_label": "fatty acid biosynthetic process",
  "term_id": "GO:0006633"
}